{
  "gene_symbol": "KRTAP19-8",
  "gene": "UniProtKB:Q3LI54",
  "term_id": "UNKNOWN:0002",
  "gene_name": "Keratin-associated protein 19-8",
  "term_label": "Unknown biological process"
}